ammonia kinase activity [GO:0047666] (molecular function) Relationships: is a type of kinase activity [GO:0016301]; is a type of phosphotransferase activity, nitrogenous group as acceptor [GO:0016775] Definition: Catalysis of the reaction: ATP + NH4 = ADP + 3 H+ + phosphoramidate. Sources: EC:2.7.3.8, RHEA:11024 Also known as: ATP:ammonia phosphotransferase activity, phosphoramidate-ADP-phosphotransferase activity, phosphoramidate-adenosine diphosphate phosphotransferase activity